{
  "gene_name": "Telomere-associated protein RIF1",
  "term_id": "GO:0000723",
  "gene": "UniProtKB:Q5UIP0",
  "term_label": "telomere maintenance",
  "gene_symbol": "RIF1"
}